amino acid binding [GO:0016597] (MF) Definition: Binding to an amino acid, organic acids containing one or more amino substituents. Sources: GOC:ai Relationships: is a type of GO:0005488 Subtypes: GO:0016594, GO:0016595, arginine binding [GO:0034618], 3-sulfino-L-alanine binding [GO:0036127], aspartate binding [GO:0070335], GO:0070728, GO:0070905, L-DOPA binding [GO:0072544], L-tyrosine binding [GO:0072545], GO:0120284, proline binding [GO:1901973], L-cysteine binding [GO:1902485]